{
  "term_id": "GO:0019814",
  "gene_name": "Immunoglobulin kappa variable 2-24",
  "gene": "UniProtKB:A0A0C4DH68",
  "gene_symbol": "IGKV2-24",
  "term_label": "immunoglobulin complex"
}